{
  "term_id": "GO:0034198",
  "gene_symbol": "KICS2",
  "term_label": "cellular response to amino acid starvation",
  "gene_name": "KICSTOR subunit 2",
  "gene": "UniProtKB:Q96MD2"
}